{
  "gene_symbol": "UPK3BL2",
  "term_id": "GO:0016020",
  "gene_name": "Uroplakin-3b-like protein 2",
  "gene": "UniProtKB:E5RIL1",
  "term_label": "membrane"
}